response to rotenone [GO:1904647] (biological process) References: PMID:18538940 Sources: GOC:TermGenie, GO_REF:0000071 Relationships: is a type of response to ketone [GO:1901654] Definition: Any process that results in a change in state or activity of a cell or an organism (in terms of movement, secretion, enzyme production, gene expression, etc.) as a result of a rotenone stimulus. Subtypes: cellular response to rotenone [GO:1904648]